galactosylgalactosylglucosylceramide beta-D-acetylgalactosaminyltransferase activity [GO:0047273] (molecular function) Relationships: is a type of acetylgalactosaminyltransferase activity [GO:0008376] Definition: Catalysis of the reaction: UDP-N-acetyl-D-galactosamine + alpha-D-galactosyl-(1->4)-beta-D-galactosyl-(1->4)-beta-D-glucosylceramide = UDP + beta-N-acetyl-D-galactosaminyl-(1->3)-alpha-D-galactosyl-(1->4)-beta-D-galactosyl-(1->4)-beta-D-glucosylceramide. Also known as: globotriosylceramide beta-1,6-N-acetylgalactosaminyltransferase activity, UDP-N-acetyl-D-galactosamine:D-galactosyl-1,4-D-galactosyl-1,4-D-glucosylceramide beta-N-acetyl-D-galactosaminyltransferase activity, UDP-N-acetyl-D-galactosamine:alpha-D-galactosyl-(1->4)-beta-D-galactosyl-(1->4)-beta-D-glucosylceramide 3III-beta-N-acetyl-D-galactosaminyltransferase activity, UDP-N-acetylgalactosamine:globotriaosylceramide beta-3-N-acetylgalactosaminyltransferase activity, UDP-N-acetylgalactosamine:globotriaosylceramide beta1,3-N-acetylgalactosaminyltransferase activity, beta-3GalNAc-T1 activity, beta3GalNAc-T1, galactosylgalactosylglucosylceramide beta-D- activity, globoside synthase activity, globoside synthetase activity, globotriaosylceramide 3-beta-N-acetylgalactosaminyltransferase activity, uridine diphosphoacetylgalactosamine-galactosylgalactosylglucosylceramide acetylgalactosaminyltransferase activity Sources: EC:2.4.1.79